{
  "gene": "UniProtKB:P58511",
  "gene_symbol": "SMIM11",
  "gene_name": "Small integral membrane protein 11",
  "term_id": "UNKNOWN:0003",
  "term_label": "Unknown cellular component"
}